ATPase dependent transmembrane transport complex [GO:0098533] (cellular component) Subtypes: ATP-binding cassette (ABC) transporter complex [GO:0043190], cation-transporting ATPase complex [GO:0090533] Relationships: is a type of transmembrane transporter complex [GO:1902495] Definition: A transmembrane protein complex that functions in ATPase dependent active transport across a membrane. Note: The location of this complex is implicit in its activity, so its location is asserted as a regular relationship rather than as a part of an intersection. Sources: GOC:dos